{
  "gene_name": "Calcium-transporting ATPase type 2C member 2",
  "gene_symbol": "ATP2C2",
  "term_label": "plasma membrane",
  "term_id": "GO:0005886",
  "gene": "UniProtKB:O75185"
}